{
  "gene_symbol": "RAD21",
  "gene": "UniProtKB:O60216",
  "term_label": "sister chromatid cohesion",
  "gene_name": "Double-strand-break repair protein rad21 homolog",
  "term_id": "GO:0007062"
}